{
  "term_label": "protein tag activity",
  "term_id": "GO:0031386",
  "gene": "UniProtKB:P62861",
  "gene_symbol": "FAU",
  "gene_name": "Ubiquitin-like FUBI-ribosomal protein eS30 fusion protein"
}